{
  "term_id": "UNKNOWN:0002",
  "gene": "UniProtKB:Q86VY9",
  "gene_name": "Transmembrane protein 200A",
  "gene_symbol": "TMEM200A",
  "term_label": "Unknown biological process"
}